regulation of metanephric mesenchymal cell migration [GO:2000589] (biological process) Subtypes: regulation of metanephric mesenchymal cell migration by platelet-derived growth factor receptor-beta signaling pathway [GO:1900238], negative regulation of metanephric mesenchymal cell migration [GO:2000590], GO:2000591 Definition: Any process that modulates the frequency, rate or extent of metanephric mesenchymal cell migration. Relationships: is a type of regulation of cell migration [GO:0030334]; regulates metanephric mesenchymal cell migration [GO:0035789] Sources: GOC:obol Also known as: regulation of metanephric mesenchyme chemotaxis